negative regulation of phosphate transmembrane transport [GO:2000186] (BP) Also known as: negative regulation of phosphate membrane transport Definition: Any process that stops, prevents, or reduces the frequency, rate or extent of phosphate transmembrane transport. Relationships: is a type of negative regulation of transmembrane transport [GO:0034763]; is a type of regulation of phosphate transmembrane transport [GO:2000185]; negatively regulates GO:0035435 Sources: GOC:obol